aryl-acylamidase activity [GO:0047680] (molecular function) Definition: Catalysis of the reaction: anilide + H2O = a carboxylate + aniline + H+. Sources: EC:3.5.1.13, RHEA:20297 Relationships: is a type of hydrolase activity, acting on carbon-nitrogen (but not peptide) bonds, in linear amides [GO:0016811] Also known as: AAA-1, AAA-2, aryl-acylamide amidohydrolase activity, brain acetylcholinesterase (is associated with AAA-2), pseudocholinesterase (associated with arylacylamidase)